{
  "gene": "UniProtKB:Q96C03",
  "term_id": "UNKNOWN:0001",
  "gene_symbol": "MIEF2",
  "gene_name": "Mitochondrial dynamics protein MID49",
  "term_label": "Unknown molecular function"
}